quinate catabolic process [GO:0019631] (biological process) Also known as: quinate breakdown, quinate catabolism, quinate degradation, quinic acid catabolic process, quinic acid catabolism Relationships: is a type of monocarboxylic acid catabolic process [GO:0072329] Sources: GOC:jl Definition: The chemical reactions and pathways resulting in the breakdown of quinate, the anion of quinic acid.